{
  "term_id": "GO:0007019",
  "gene_symbol": "STMN3",
  "gene": "UniProtKB:Q9NZ72",
  "gene_name": "Stathmin-3",
  "term_label": "microtubule depolymerization"
}